CCAAT-binding factor complex [GO:0016602] (cellular component) Definition: A heteromeric transcription factor complex that binds to the CCAAT-box upstream of promoters; functions as both an activator and a repressor, depending on its interacting cofactors. Typically trimeric consisting of NFYA, NFYB and NFYC subunits. In Saccharomyces, it activates the transcription of genes in response to growth in a nonfermentable carbon source and consists of four known subunits: HAP2, HAP3, HAP4 and HAP5. References: PMID:7828851 Sources: GOC:bhm Also known as: CBF complex, NF-Y transcription factor complex, nuclear transcription factor Y complex Relationships: is a type of RNA polymerase II transcription regulator complex [GO:0090575]